{
  "gene": "UniProtKB:P25106",
  "term_id": "GO:0007204",
  "gene_name": "Atypical chemokine receptor 3",
  "term_label": "positive regulation of cytosolic calcium ion concentration",
  "gene_symbol": "ACKR3"
}